adhesion receptor-mediated virion attachment to host cell [GO:0098671] (biological process) Definition: The process by which a virion attaches to a host cell by binding to a receptor on the host cell surface that does not mediate or trigger entry into the host cell. This binding is typically reversible and enhances significantly infectivity by concentrating the virus in the vicinity of its entry receptors, or bringing it to an organ in which its target cells are located. References: PMID:18351291 Sources: VZ:3943 Also known as: viral attachment to host adhesion receptor Relationships: is a type of receptor-mediated virion attachment to host cell [GO:0046813] Subtypes: receptor-mediated bacteriophage reversible attachment to host cell [GO:0098001]